{
  "term_id": "GO:0005615",
  "gene": "UniProtKB:Q6JVE5",
  "term_label": "extracellular space",
  "gene_name": "Epididymal-specific lipocalin-12",
  "gene_symbol": "LCN12"
}